{
  "gene": "UniProtKB:O94907",
  "term_id": "GO:0090090",
  "gene_symbol": "DKK1",
  "gene_name": "Dickkopf-related protein 1",
  "term_label": "negative regulation of canonical Wnt signaling pathway"
}